anterograde trans-synaptic signaling [GO:0098916] (biological process) Sources: GOC:dos Subtypes: GO:0007268, anterograde trans-synaptic signaling by nitric oxide [GO:0098940], anterograde trans-synaptic signaling by trans-synaptic protein complex [GO:0098941] Definition: Cell-cell signaling from pre to post-synapse, across the synaptic cleft. Relationships: is a type of trans-synaptic signaling [GO:0099537]